{
  "term_label": "Unknown biological process",
  "term_id": "UNKNOWN:0002",
  "gene": "UniProtKB:O14519",
  "gene_name": "Cyclin-dependent kinase 2-associated protein 1",
  "gene_symbol": "CDK2AP1"
}